{
  "gene_name": "Putative adhesion G protein-coupled receptor E4P",
  "term_label": "plasma membrane",
  "gene": "UniProtKB:Q86SQ3",
  "gene_symbol": "ADGRE4P",
  "term_id": "GO:0005886"
}